{
  "term_label": "peroxisome",
  "gene": "UniProtKB:Q9UJ83",
  "gene_symbol": "HACL1",
  "term_id": "GO:0005777",
  "gene_name": "2-hydroxyacyl-CoA lyase 1"
}